brown fat cell proliferation [GO:0070342] (biological process) Definition: The multiplication or reproduction of brown fat cells by cell division, resulting in the expansion of their population. A brown fat cell is a fat cell found the thermogenic form of adipose tissue found in newborns of many species. Relationships: is a type of fat cell proliferation [GO:0070341] Sources: CL:0000449, GOC:mah, GOC:sl Regulation: regulated by regulation of brown fat cell proliferation [GO:0070347]; negatively regulated by negative regulation of brown fat cell proliferation [GO:0070348]; positively regulated by positive regulation of brown fat cell proliferation [GO:0070349] Also known as: brown adipocyte proliferation, brown adipose cell proliferation